MutSbeta complex [GO:0032302] (CC) Relationships: is a type of mismatch repair complex [GO:0032300]; is a type of nuclear protein-containing complex [GO:0140513] References: PMID:11005803 Also known as: MMR complex, MSH2/MSH3 complex Definition: A heterodimer involved in binding to and correcting insertion/deletion mutations. In human the complex consists of two subunits, MSH2 and MSH3.